{
  "gene_name": "Zinc finger protein 428",
  "gene": "UniProtKB:Q96B54",
  "gene_symbol": "ZNF428",
  "term_id": "UNKNOWN:0003",
  "term_label": "Unknown cellular component"
}